{
  "term_label": "ATP binding",
  "term_id": "GO:0005524",
  "gene_symbol": "ABCF1",
  "gene_name": "ATP-binding cassette sub-family F member 1",
  "gene": "UniProtKB:Q8NE71"
}